response to G2 DNA damage checkpoint signaling [GO:0072426] (biological process) Subtypes: GO:0072435 Definition: A process that occurs in response to signals generated as a result of G2/M transition DNA damage checkpoint signaling. Relationships: is a type of GO:0072423 Sources: GOC:mtg_cell_cycle Regulation: regulated by regulation of response to G2 DNA damage checkpoint signaling [GO:1902157]; positively regulated by positive regulation of response to G2 DNA damage checkpoint signaling [GO:1902158] Also known as: G2/M transition DNA damage checkpoint effector process, response to signal involved in G2/M transition DNA damage checkpoint